{
  "gene_symbol": "ANKIB1",
  "gene": "UniProtKB:Q9P2G1",
  "term_id": "GO:0061630",
  "gene_name": "Ankyrin repeat and IBR domain-containing protein 1",
  "term_label": "ubiquitin protein ligase activity"
}